cell adhesion involved in biofilm formation [GO:0043708] (biological process) Definition: The attachment of a cell to a solid substrate, via cell adhesion molecules, contributing to the formation of a biofilm. Sources: GOC:dph, GOC:jl, GOC:tb Also known as: cell adhesion during biofilm formation Relationships: is a type of cell-substrate adhesion [GO:0031589]; is part of submerged biofilm formation [GO:0090605] Subtypes: GO:0043709, cell adhesion involved in multi-species biofilm formation [GO:0043710]